{
  "gene_symbol": "ECE2",
  "term_label": "protein processing",
  "gene": "UniProtKB:P0DPD6",
  "term_id": "GO:0016485",
  "gene_name": "Endothelin-converting enzyme 2"
}